{
  "gene_symbol": "SRSF9",
  "gene_name": "Serine_arginine-rich splicing factor 9",
  "term_label": "nuclear speck",
  "term_id": "GO:0016607",
  "gene": "UniProtKB:Q13242"
}